ribonucleoprotein complex biogenesis [GO:0022613] (biological process) Definition: A cellular process that results in the biosynthesis of constituent macromolecules, assembly, and arrangement of constituent parts of a complex containing RNA and proteins. Includes the biosynthesis of the constituent RNA and protein molecules, and those macromolecular modifications that are involved in synthesis or assembly of the ribonucleoprotein complex. Relationships: is a type of cellular component biogenesis [GO:0044085] Subtypes: GO:0042254, ribosomal large subunit biogenesis [GO:0042273], GO:0042274 Sources: GOC:isa_complete, GOC:mah Also known as: RNA-protein complex biogenesis, ribonucleoprotein complex biogenesis and assembly